4-alpha-hydroxytetrahydrobiopterin dehydratase activity [GO:0008124] (molecular function) Also known as: 4a-hydroxytetrahydrobiopterin dehydratase activity, pterin-4-alpha-carbinolamine dehydratase activity, pterin-4a-carbinolamine dehydratase activity, (6R)-6-(L-erythro-1,2-dihydroxypropyl)-5,6,7,8-tetrahydro-4a-hydroxypterin hydro-lyase [(6R)-6-(L-erythro-1,2-dihydroxypropyl)-7,8-dihydro-6H-pterin-forming], 4-alpha-hydroxy-tetrahydropterin dehydratase activity, 4a-hydroxytetrahydrobiopterin hydro-lyase activity, 4alpha-hydroxy-tetrahydropterin dehydratase activity, pterin-4alpha-carbinolamine dehydratase activity, tetrahydrobiopterin dehydratase activity Definition: Catalysis of the reaction: (6R)-6-(L-erythro-1,2-dihydroxypropyl)-5,6,7,8-tetrahydro-4a-hydroxypterin = (6R)-6-(L-erythro-1,2-dihydroxypropyl)-7,8-dihydro-6H-pterin + H2O. Sources: EC:4.2.1.96, RHEA:11920 Relationships: is a type of hydro-lyase activity [GO:0016836]